caecum development [GO:1903700] (biological process) Definition: The process whose specific outcome is the progression of a caecum over time, from its formation to the mature structure. Also known as: cecum development, intestinum crassum caecum development, caeca development, ceca development, blind intestine development, blindgut development, intestinum caecum development, intestinum crassum cecum development Sources: GOC:TermGenie, GO_REF:0000094, ISBN:0-683-40008-8 Relationships: is a type of GO:0048856